{
  "gene_name": "Cytoglobin",
  "term_id": "UNKNOWN:0003",
  "gene": "UniProtKB:Q8WWM9",
  "term_label": "Unknown cellular component",
  "gene_symbol": "CYGB"
}